{
  "gene_symbol": "NSD1",
  "gene": "UniProtKB:Q96L73",
  "gene_name": "Histone-lysine N-methyltransferase, H3 lysine-36 specific",
  "term_id": "GO:0006355",
  "term_label": "regulation of DNA-templated transcription"
}